{
  "gene": "UniProtKB:Q9P1G2",
  "gene_symbol": "RBM12B-AS1",
  "term_label": "Unknown cellular component",
  "term_id": "UNKNOWN:0003",
  "gene_name": "Putative uncharacterized protein encoded by RBM12B-AS1"
}